{
  "gene": "UniProtKB:Q13609",
  "gene_symbol": "DNASE1L3",
  "term_id": "GO:0010623",
  "term_label": "programmed cell death involved in cell development",
  "gene_name": "Deoxyribonuclease gamma"
}